{
  "gene": "UniProtKB:Q15691",
  "term_label": "protein localization to microtubule",
  "gene_symbol": "MAPRE1",
  "term_id": "GO:0035372",
  "gene_name": "Microtubule-associated protein RP_EB family member 1"
}